{
  "gene_name": "V-type proton ATPase subunit S1-like protein",
  "term_label": "Unknown biological process",
  "gene_symbol": "ATP6AP1L",
  "term_id": "UNKNOWN:0002",
  "gene": "UniProtKB:Q52LC2"
}